{
  "term_label": "ATP hydrolysis activity",
  "gene_name": "Kinesin-like protein KIF27",
  "gene": "UniProtKB:Q86VH2",
  "gene_symbol": "KIF27",
  "term_id": "GO:0016887"
}